positive regulation of protein localization to nucleolus [GO:1904751] (biological process) Also known as: positive regulation of protein localisation in nucleolus, positive regulation of protein localisation to nucleolus, positive regulation of protein localization in nucleolus, up regulation of protein localisation in nucleolus, up regulation of protein localisation to nucleolus, up regulation of protein localization in nucleolus, up regulation of protein localization to nucleolus, up-regulation of protein localisation in nucleolus, up-regulation of protein localisation to nucleolus, up-regulation of protein localization in nucleolus, up-regulation of protein localization to nucleolus, upregulation of protein localisation in nucleolus, upregulation of protein localisation to nucleolus, upregulation of protein localization in nucleolus, upregulation of protein localization to nucleolus, activation of protein localisation in nucleolus, activation of protein localisation to nucleolus, activation of protein localization in nucleolus, activation of protein localization to nucleolus References: PMID:24415760 Sources: GOC:BHF, GOC:BHF_telomere, GOC:TermGenie, GOC:nc, GO_REF:0000058 Definition: Any process that activates or increases the frequency, rate or extent of protein localization to nucleolus. Relationships: is a type of positive regulation of protein localization to nucleus [GO:1900182]; is a type of regulation of protein localization to nucleolus [GO:1904749]; positively regulates protein localization to nucleolus [GO:1902570]